{
  "gene_symbol": "ZNF304",
  "gene": "UniProtKB:Q9HCX3",
  "term_id": "GO:0006357",
  "term_label": "regulation of transcription by RNA polymerase II",
  "gene_name": "Zinc finger protein 304"
}